bacterial-type flagellum basal body, proximal rod [GO:0009429] (cellular component) Definition: The portion of the central rod of the bacterial-type flagellar basal body that is proximal to the cell membrane; the proximal rod connects the distal rod to the flagellar motor. References: PMID:10572114, PMID:11133968, PMID:12624192 Sources: GOC:cilia, GOC:mtg_sensu Relationships: is a type of GO:0110165; is part of GO:0030694 Also known as: flagellar basal body, proximal rod, flagellin-based flagellum basal body, proximal rod